{
  "gene_name": "Heat shock factor protein 2",
  "gene_symbol": "HSF2",
  "term_id": "GO:0003700",
  "gene": "UniProtKB:Q03933",
  "term_label": "DNA-binding transcription factor activity"
}